{
  "gene_name": "Prolactin",
  "gene_symbol": "PRL",
  "term_id": "GO:0005148",
  "gene": "UniProtKB:P01236",
  "term_label": "prolactin receptor binding"
}